{
  "gene_name": "Protein BRICK1",
  "gene": "UniProtKB:Q8WUW1",
  "term_id": "UNKNOWN:0001",
  "gene_symbol": "BRK1",
  "term_label": "Unknown molecular function"
}